{
  "gene_symbol": "LY9",
  "term_label": "external side of plasma membrane",
  "term_id": "GO:0009897",
  "gene_name": "T-lymphocyte surface antigen Ly-9",
  "gene": "UniProtKB:Q9HBG7"
}